{
  "term_label": "plasma membrane",
  "term_id": "GO:0005886",
  "gene": "UniProtKB:P06127",
  "gene_symbol": "CD5",
  "gene_name": "T-cell surface glycoprotein CD5"
}